{
  "gene": "UniProtKB:O95521",
  "term_label": "ubiquitin-like ligase-substrate adaptor activity",
  "gene_symbol": "PRAMEF1",
  "gene_name": "PRAME family member 1",
  "term_id": "GO:1990756"
}